{
  "term_label": "Unknown biological process",
  "gene": "UniProtKB:Q9NQ39",
  "term_id": "UNKNOWN:0002",
  "gene_symbol": "RPS10P5",
  "gene_name": "Putative ribosomal protein eS10-like"
}